{
  "gene": "UniProtKB:P0C854",
  "gene_name": "Putative cat eye syndrome critical region protein 9",
  "term_label": "Unknown biological process",
  "term_id": "UNKNOWN:0002",
  "gene_symbol": "CECR9"
}